{
  "term_label": "cyclosporin A binding",
  "gene": "UniProtKB:P23284",
  "gene_name": "Peptidyl-prolyl cis-trans isomerase B",
  "term_id": "GO:0016018",
  "gene_symbol": "PPIB"
}